granulosa cell apoptotic process [GO:1904700] (biological process) Also known as: granulosa cell of ovary apoptotic process, granulosa cell apoptosis, granulosa cell of ovary apoptosis References: PMID:19208546 Sources: GOC:TermGenie, GO_REF:0000085 Definition: Any apoptotic process in a granulosa cell. Regulation: regulated by regulation of granulosa cell apoptotic process [GO:1904708]; negatively regulated by GO:1904709; positively regulated by positive regulation of granulosa cell apoptotic process [GO:1904710] Relationships: is a type of epithelial cell apoptotic process [GO:1904019]